{
  "gene_symbol": "UBE4A",
  "term_label": "cytoplasm",
  "gene_name": "Ubiquitin conjugation factor E4 A",
  "term_id": "GO:0005737",
  "gene": "UniProtKB:Q14139"
}